{
  "gene": "UniProtKB:Q9NRD8",
  "gene_symbol": "DUOX2",
  "term_id": "GO:0005886",
  "gene_name": "Dual oxidase 2",
  "term_label": "plasma membrane"
}